{
  "gene": "UniProtKB:Q8NC51",
  "gene_name": "SERPINE1 mRNA-binding protein 1",
  "gene_symbol": "SERBP1",
  "term_id": "UNKNOWN:0002",
  "term_label": "Unknown biological process"
}